{
  "gene_symbol": "CD274",
  "gene_name": "Programmed cell death 1 ligand 1",
  "term_id": "GO:0007166",
  "gene": "UniProtKB:Q9NZQ7",
  "term_label": "cell surface receptor signaling pathway"
}